Mo-molybdopterin cofactor metabolic process [GO:0019720] (biological process) Also known as: Moco metabolic process, Moco metabolism, Mo-molybdopterin cofactor metabolism Relationships: is a type of molybdopterin cofactor metabolic process [GO:0043545] Subtypes: Mo-molybdopterin cofactor biosynthetic process [GO:0006777], GO:0032326 References: PMID:23539623, PMID:35956883 Definition: The chemical reactions and pathways involving the Mo-molybdopterin cofactor, essential for the catalytic activity of some enzymes. The cofactor consists of a mononuclear molybdenum (Mo) ion coordinated by one or two molybdopterin ligands.